{
  "term_id": "UNKNOWN:0003",
  "gene_symbol": "LOC728743",
  "gene": "UniProtKB:B7ZLF3",
  "term_label": "Unknown cellular component",
  "gene_name": "C2H2-type domain-containing protein"
}